turning behavior involved in mating [GO:0034607] (biological process) Regulation: regulated by regulation of turning behavior involved in mating [GO:0061094]; positively regulated by positive regulation of turning behavior involved in mating [GO:0061095]; negatively regulated by negative regulation of turning behavior involved in mating [GO:0061096] Definition: The sharp ventral turn performed by the male as he approaches either the hermaphrodite head or tail, whilst trying to locate his partner's vulva. Turning occurs via a sharp ventral coil of the male's tail. References: PMID:18050467 Sources: WB_REF:WBPaper00002109 Relationships: is a type of male mating behavior [GO:0060179] Also known as: turning behavior during mating